ureidoglycolate dehydrogenase activity [GO:0009040] (molecular function) Also known as: (S)-ureidoglycolate:NAD(P)+ oxidoreductase activity Definition: Catalysis of the reaction: (S)-ureidoglycolate + NAD(P)+ = oxalureate + NAD(P)H + H+. References: PMID:23284870 Sources: EC:1.1.1.154 Relationships: is a type of oxidoreductase activity, acting on the CH-OH group of donors, NAD or NADP as acceptor [GO:0016616]